{
  "term_label": "regulation of release of sequestered calcium ion into cytosol by sarcoplasmic reticulum",
  "gene": "UniProtKB:P0DP25",
  "gene_symbol": "CALM3",
  "term_id": "GO:0010880",
  "gene_name": "Calmodulin-3"
}